{
  "gene_name": "ATPase MORC2",
  "gene_symbol": "MORC2",
  "term_id": "UNKNOWN:0001",
  "term_label": "Unknown molecular function",
  "gene": "UniProtKB:Q9Y6X9"
}